{
  "term_id": "GO:0006541",
  "gene_name": "CAD protein",
  "term_label": "glutamine metabolic process",
  "gene": "UniProtKB:P27708",
  "gene_symbol": "CAD"
}